{
  "term_id": "GO:0005737",
  "gene_symbol": "CDC25B",
  "gene_name": "M-phase inducer phosphatase 2",
  "gene": "UniProtKB:P30305",
  "term_label": "cytoplasm"
}